positive regulation of protein localization to spindle pole body [GO:1902365] (biological process) Definition: Any process that activates or increases the frequency, rate or extent of protein localization to spindle pole body. References: PMID:21131906 Sources: GOC:TermGenie Subtypes: positive regulation of protein localization to meiotic spindle pole body [GO:0140434] Also known as: positive regulation of protein localisation to spindle pole body, up regulation of protein localisation to spindle pole body, up regulation of protein localization to spindle pole body, up-regulation of protein localisation to spindle pole body, up-regulation of protein localization to spindle pole body, upregulation of protein localisation to spindle pole body, upregulation of protein localization to spindle pole body, activation of protein localisation to spindle pole body, activation of protein localization to spindle pole body Relationships: is a type of GO:1902363; is a type of positive regulation of protein localization [GO:1903829]; positively regulates GO:0071988